{
  "gene_symbol": "MFSD1",
  "term_id": "UNKNOWN:0001",
  "gene_name": "Major facilitator superfamily domain-containing protein 1",
  "term_label": "Unknown molecular function",
  "gene": "UniProtKB:Q9H3U5"
}